{
  "gene_name": "NUT family member 2A",
  "term_id": "UNKNOWN:0003",
  "gene_symbol": "NUTM2A",
  "gene": "UniProtKB:Q8IVF1",
  "term_label": "Unknown cellular component"
}